{
  "gene_symbol": "ING2",
  "term_label": "Unknown molecular function",
  "term_id": "UNKNOWN:0001",
  "gene_name": "Inhibitor of growth protein 2",
  "gene": "UniProtKB:Q9H160"
}